FAT10 transferase activity [GO:0019775] (MF) Subtypes: FAT10 conjugating enzyme activity [GO:0061652], FAT10 ligase activity [GO:0061661] Relationships: is a type of GO:0019787 Definition: Catalysis of the transfer of FAT10 from one protein to another via the reaction X-FAT10 + Y = Y-FAT10 + X, where both X-FAT10 and Y-FAT10 are covalent linkages. References: PMID:12826404 Sources: GOC:dph, GOC:mah Also known as: FAT10 conjugating enzyme activity